{
  "gene_symbol": "OR5B17",
  "term_id": "GO:0004984",
  "gene": "UniProtKB:Q8NGF7",
  "term_label": "olfactory receptor activity",
  "gene_name": "Olfactory receptor 5B17"
}